{
  "gene_symbol": "NAP1L5",
  "gene": "UniProtKB:Q96NT1",
  "gene_name": "Nucleosome assembly protein 1-like 5",
  "term_id": "UNKNOWN:0001",
  "term_label": "Unknown molecular function"
}